{
  "gene_name": "Sickle tail protein homolog",
  "term_id": "GO:0005737",
  "term_label": "cytoplasm",
  "gene_symbol": "KIAA1217",
  "gene": "UniProtKB:Q5T5P2"
}